{
  "gene": "UniProtKB:Q8IVF6",
  "term_label": "Unknown molecular function",
  "term_id": "UNKNOWN:0001",
  "gene_name": "Ankyrin repeat domain-containing protein 18A",
  "gene_symbol": "ANKRD18A"
}